{
  "gene_symbol": "OR2T5",
  "gene_name": "Olfactory receptor 2T5",
  "term_id": "GO:0005886",
  "gene": "UniProtKB:Q6IEZ7",
  "term_label": "plasma membrane"
}